positive regulation of renal albumin absorption [GO:2000534] (biological process) Sources: GOC:obol, GOC:yaf Relationships: is a type of positive regulation of multicellular organismal process [GO:0051240]; is a type of GO:2000532; positively regulates GO:0097018 Definition: Any process that activates or increases the frequency, rate or extent of renal albumin absorption.